{
  "gene_name": "Follicle-stimulating hormone receptor",
  "term_id": "GO:0007189",
  "term_label": "adenylate cyclase-activating G protein-coupled receptor signaling pathway",
  "gene_symbol": "FSHR",
  "gene": "UniProtKB:P23945"
}